negative regulation of actin filament polymerization [GO:0030837] (biological process) Subtypes: GO:0051693 Note: Note that this term was split from 'negative regulation of actin polymerization and/or depolymerization ; GO:0045757' (sibling term 'negative regulation of actin depolymerization ; GO:0030835'). Definition: Any process that stops, prevents, or reduces the frequency, rate or extent of actin polymerization. Also known as: negative regulation of actin polymerization and/or depolymerization, down regulation of actin filament polymerization, down-regulation of actin filament polymerization, downregulation of actin filament polymerization, negative regulation of actin polymerization, inhibition of actin filament polymerization Relationships: is_a regulation of actin filament polymerization [GO:0030833]; is a type of negative regulation of protein polymerization [GO:0032272]; is a type of negative regulation of cytoskeleton organization [GO:0051494]; is a type of negative regulation of supramolecular fiber organization [GO:1902904]; negatively regulates actin filament polymerization [GO:0030041] Sources: GOC:mah